catechol-containing compound metabolic process [GO:0009712] (biological process) Definition: The chemical reactions and pathways involving a compound containing a pyrocatechol (1,2-benzenediol) nucleus or substituent. Sources: GOC:sm, ISBN:0198547684 Also known as: catechol metabolic process, catechol metabolism Relationships: is a type of phenol-containing compound metabolic process [GO:0018958] Subtypes: catecholamine metabolic process [GO:0006584], GO:0009713, L-tryptophan catabolic process to catechol [GO:0019444], toluene oxidation to catechol [GO:0019604], catechol-containing compound catabolic process [GO:0019614], 3,4-dihydroxybenzoate metabolic process [GO:0046278], violaceol I metabolic process [GO:1900588], GO:1900591, cordyol C metabolic process [GO:1900797]